{
  "term_label": "membrane",
  "gene_symbol": "SGTB",
  "term_id": "GO:0016020",
  "gene_name": "Small glutamine-rich tetratricopeptide repeat-containing protein beta",
  "gene": "UniProtKB:Q96EQ0"
}